{
  "gene": "UniProtKB:P0C263",
  "term_label": "Unknown cellular component",
  "term_id": "UNKNOWN:0003",
  "gene_name": "Serine_threonine-protein kinase SBK2",
  "gene_symbol": "SBK2"
}